{
  "gene_name": "NIPA-like protein 3",
  "term_label": "membrane",
  "gene_symbol": "NIPAL3",
  "gene": "UniProtKB:Q6P499",
  "term_id": "GO:0016020"
}